regulation of somatic stem cell division [GO:1904675] (biological process) Definition: Any process that modulates the frequency, rate or extent of somatic stem cell division. Also known as: regulation of somatic stem cell renewal Relationships: is a type of regulation of stem cell division [GO:2000035]; RO_0002211 somatic stem cell division [GO:0048103] References: PMID:19409607 Sources: GOC:BHF, GOC:BHF_miRNA, GOC:TermGenie, GOC:rph, GO_REF:0000058 Subtypes: negative regulation of somatic stem cell division [GO:1904676], GO:1904677